gut granule lumen [GO:0044842] (cellular component) Relationships: is a type of intracellular organelle lumen [GO:0070013]; is part of gut granule [GO:0044840] Definition: The lumen of a gut granule, a lysosome-related organelle contained within the intestinal cells of the nematode C. elegans. References: PMID:22916203, PMID:24204312 Sources: GOC:kmv